{
  "term_id": "GO:0006357",
  "term_label": "regulation of transcription by RNA polymerase II",
  "gene_symbol": "IKZF3",
  "gene": "UniProtKB:Q9UKT9",
  "gene_name": "Zinc finger protein Aiolos"
}